{
  "term_label": "GTPase activator activity",
  "term_id": "GO:0005096",
  "gene_name": "Rho GTPase-activating protein 40",
  "gene_symbol": "ARHGAP40",
  "gene": "UniProtKB:Q5TG30"
}